{
  "gene": "UniProtKB:Q5SXM1",
  "gene_name": "Zinc finger protein 678",
  "gene_symbol": "ZNF678",
  "term_id": "GO:0000978",
  "term_label": "RNA polymerase II cis-regulatory region sequence-specific DNA binding"
}